{
  "gene_symbol": "LGALS8",
  "term_label": "cytoplasm",
  "gene_name": "Galectin-8",
  "term_id": "GO:0005737",
  "gene": "UniProtKB:O00214"
}